response to interleukin-3 [GO:0036015] (biological process) Definition: Any process that results in a change in state or activity of a cell or an organism (in terms of movement, secretion, enzyme production, gene expression, etc.) as a result of an interleukin-3 stimulus. Sources: GOC:yaf Also known as: response to IL-3 Relationships: is a type of response to cytokine [GO:0034097] Subtypes: cellular response to interleukin-3 [GO:0036016]